{
  "gene_name": "Kinase D-interacting substrate of 220 kDa",
  "term_label": "protein kinase regulator activity",
  "term_id": "GO:0019887",
  "gene": "UniProtKB:Q9ULH0",
  "gene_symbol": "KIDINS220"
}